{
  "gene_name": "Ataxin-10",
  "gene": "UniProtKB:Q9UBB4",
  "gene_symbol": "ATXN10",
  "term_label": "neuron projection development",
  "term_id": "GO:0031175"
}